phosphatidylglycerol biosynthetic process [GO:0006655] (biological process) Regulation: regulated by regulation of phosphatidylglycerol biosynthetic process [GO:1901351]; negatively regulated by negative regulation of phosphatidylglycerol biosynthetic process [GO:1901352]; positively regulated by GO:1901353 Relationships: is a type of phosphatidylglycerol metabolic process [GO:0046471]; is a type of glycerophospholipid biosynthetic process [GO:0046474] Also known as: phosphatidylglycerol anabolism, phosphatidylglycerol biosynthesis, phosphatidylglycerol formation, phosphatidylglycerol synthesis Subtypes: GO:0032049 Definition: The chemical reactions and pathways resulting in the formation of phosphatidylglycerols, any of a class of phospholipids in which the phosphatidyl group is esterified to the hydroxyl group of glycerol. Sources: ISBN:0198506732